mitotic nuclear membrane microtubule tethering complex [GO:0106084] (CC) Definition: A protein complex capable of interacting with the spindle pole body and the nuclear envelope, in order to embed the spindle pole body in the nuclear envelope at fusion sites of the inner and outer nuclear membrane. References: PMID:28356353 Sources: GOC:lnp Relationships: is a type of nuclear membrane microtubule tethering complex [GO:0106094] Note: In S. cerevisae Mps2-Bpb1 is the membrane anchor sub complex and Spc29 is the spindle pole body linker molecule. Also known as: nuclear membrane mitotic spindle pole body tethering complex, Mps2-Bbp1-Spc29 complex